{
  "term_id": "GO:0034499",
  "gene_name": "GRIP and coiled-coil domain-containing protein 2",
  "gene": "UniProtKB:Q8IWJ2",
  "gene_symbol": "GCC2",
  "term_label": "late endosome to Golgi transport"
}